preantral ovarian follicle growth [GO:0001546] (biological process) Sources: https://www.ncbi.nlm.nih.gov/books/NBK279054/ Definition: Increase in size of follicles surrounded by two or more layers of granulosa cells up to the onset of antrum formation. Relationships: is a type of ovulation cycle process [GO:0022602]; is a type of developmental growth [GO:0048589]; is part of ovarian follicle development [GO:0001541]; is part of multi-layer follicle stage [GO:0048162]